{
  "gene_name": "Heat shock protein beta-6",
  "term_id": "GO:0009408",
  "term_label": "response to heat",
  "gene": "UniProtKB:O14558",
  "gene_symbol": "HSPB6"
}